negative regulation of auditory receptor cell fate specification [GO:0009999] (biological process) Definition: Any process that restricts, stops or prevents a cell from specifying into an auditory hair cell. Sources: GOC:go_curators Also known as: down regulation of auditory receptor cell fate specification, down-regulation of auditory receptor cell fate specification, downregulation of auditory receptor cell fate specification, negative regulation of auditory hair cell fate specification, suppression of auditory receptor cell fate, suppression of hair cell fate, inhibition of auditory receptor cell fate specification Relationships: is a type of negative regulation of cell fate specification [GO:0009996]; is a type of regulation of inner ear auditory receptor cell fate specification [GO:0042669]; is a type of negative regulation of inner ear auditory receptor cell differentiation [GO:0045608]; negatively regulates auditory receptor cell fate specification [GO:0042667]